interferon-beta production [GO:0032608] (biological process) Definition: The appearance of interferon-beta due to biosynthesis or secretion following a cellular stimulus, resulting in an increase in its intracellular or extracellular levels. Relationships: is_a type I interferon production [GO:0032606] Also known as: IFN-beta production, IFNB production, interferon-beta biosynthetic process, interferon-beta secretion Regulation: regulated by regulation of interferon-beta production [GO:0032648]; negatively regulated by negative regulation of interferon-beta production [GO:0032688]; positively regulated by positive regulation of interferon-beta production [GO:0032728] Note: Note that this term is in the subset of terms that should not be used for direct gene product annotation. Instead, select one of the 'regulation' children terms. References: PMID:15546383 Sources: GOC:mah